{
  "term_id": "GO:0006491",
  "gene_name": "Beta-hexosaminidase subunit alpha",
  "gene_symbol": "HEXA",
  "gene": "UniProtKB:P06865",
  "term_label": "N-glycan processing"
}